{
  "term_label": "protein localization to cell-cell junction",
  "gene_symbol": "CGNL1",
  "gene_name": "Cingulin-like protein 1",
  "term_id": "GO:0150105",
  "gene": "UniProtKB:Q0VF96"
}